{
  "gene_name": "Tribbles homolog 1",
  "term_id": "GO:0005634",
  "gene_symbol": "TRIB1",
  "term_label": "nucleus",
  "gene": "UniProtKB:Q96RU8"
}